{
  "term_id": "GO:1900158",
  "gene": "UniProtKB:Q8N5W9",
  "term_label": "negative regulation of bone mineralization involved in bone maturation",
  "gene_symbol": "RFLNB",
  "gene_name": "Refilin-B"
}